{
  "gene_symbol": "OR6S1",
  "gene_name": "Olfactory receptor 6S1",
  "term_id": "GO:0004984",
  "gene": "UniProtKB:Q8NH40",
  "term_label": "olfactory receptor activity"
}